{
  "term_id": "GO:0005634",
  "term_label": "nucleus",
  "gene_name": "Cytokine receptor-like factor 3",
  "gene": "UniProtKB:Q8IUI8",
  "gene_symbol": "CRLF3"
}